{
  "gene_name": "Glycogen synthase kinase-3 alpha",
  "term_id": "GO:0005634",
  "term_label": "nucleus",
  "gene_symbol": "GSK3A",
  "gene": "UniProtKB:P49840"
}